{
  "gene_symbol": "HOXA11",
  "term_id": "GO:0005634",
  "gene": "UniProtKB:P31270",
  "gene_name": "Homeobox protein Hox-A11",
  "term_label": "nucleus"
}